{
  "term_id": "GO:0000122",
  "gene_name": "Methyl-CpG-binding domain protein 3-like 2",
  "gene": "UniProtKB:Q8NHZ7",
  "gene_symbol": "MBD3L2",
  "term_label": "negative regulation of transcription by RNA polymerase II"
}